{
  "gene": "UniProtKB:Q9BUH6",
  "term_label": "nonhomologous end joining complex",
  "term_id": "GO:0070419",
  "gene_symbol": "PAXX",
  "gene_name": "Protein PAXX"
}